{
  "gene_symbol": "TMOD2",
  "term_id": "GO:0006936",
  "gene_name": "Tropomodulin-2",
  "gene": "UniProtKB:Q9NZR1",
  "term_label": "muscle contraction"
}